{
  "gene": "UniProtKB:P42566",
  "term_id": "GO:0030674",
  "gene_name": "Epidermal growth factor receptor substrate 15",
  "term_label": "protein-macromolecule adaptor activity",
  "gene_symbol": "EPS15"
}